{
  "gene": "UniProtKB:Q9C0H6",
  "term_id": "GO:1990756",
  "gene_symbol": "KLHL4",
  "term_label": "ubiquitin-like ligase-substrate adaptor activity",
  "gene_name": "Kelch-like protein 4"
}